{
  "gene_symbol": "AGL",
  "gene": "UniProtKB:P35573",
  "gene_name": "Glycogen debranching enzyme",
  "term_label": "amylo-alpha-1,6-glucosidase activity",
  "term_id": "GO:0004135"
}